{
  "gene_name": "High mobility group protein 20A",
  "term_id": "UNKNOWN:0001",
  "term_label": "Unknown molecular function",
  "gene_symbol": "HMG20A",
  "gene": "UniProtKB:Q9NP66"
}